{
  "gene_symbol": "TRAPPC5",
  "gene": "UniProtKB:Q8IUR0",
  "term_label": "TRAPPII protein complex",
  "gene_name": "Trafficking protein particle complex subunit 5",
  "term_id": "GO:1990071"
}